alpha6-beta1 integrin-CD151 complex [GO:0071059] (CC) Relationships: is a type of GO:0098797 Definition: A protein complex that consists of an alpha6-beta1 integrin complex bound to the tetraspanin CD151. References: PMID:11884516 Also known as: ITGA6-ITGB1-CD151 complex